xylitol oxidase activity [GO:0050582] (molecular function) Sources: EC:1.1.3.41 Relationships: is a type of oxidoreductase activity, acting on the CH-OH group of donors, oxygen as acceptor [GO:0016899] Definition: Catalysis of the reaction: xylitol + O2 = xylose + H2O2. Xylitol (five carbons) and sorbitol (6 carbons) are the preferred substrates. Also known as: xylitol:oxygen oxidoreductase activity